galactose-6-phosphate isomerase activity [GO:0050044] (molecular function) Also known as: D-galactose-6-phosphate aldose-ketose-isomerase activity, D-galactose-6-phosphate ketol-isomerase activity Definition: Catalysis of the reaction: D-galactose 6-phosphate = D-tagatose 6-phosphate. Sources: EC:5.3.1.26, RHEA:13033 Relationships: is a type of intramolecular oxidoreductase activity, interconverting aldoses and ketoses [GO:0016861]